{
  "term_id": "GO:0019901",
  "gene": "UniProtKB:P0DUD4",
  "term_label": "protein kinase binding",
  "gene_name": "Putative speedy protein E15",
  "gene_symbol": "SPDYE15"
}